{
  "gene_symbol": "RGPD3",
  "term_label": "SUMO transferase activity",
  "gene_name": "RanBP2-like and GRIP domain-containing protein 3",
  "term_id": "GO:0019789",
  "gene": "UniProtKB:A6NKT7"
}